{
  "gene": "UniProtKB:Q9BRX9",
  "gene_symbol": "WDR83",
  "term_label": "mRNA splicing, via spliceosome",
  "gene_name": "WD repeat domain-containing protein 83",
  "term_id": "GO:0000398"
}